{
  "gene": "UniProtKB:P08754",
  "gene_name": "Guanine nucleotide-binding protein G(i) subunit alpha-3",
  "term_id": "GO:0031683",
  "gene_symbol": "GNAI3",
  "term_label": "G-protein beta/gamma-subunit complex binding"
}